{
  "term_id": "GO:0005634",
  "gene": "UniProtKB:P0CB48",
  "gene_symbol": "UBTFL6",
  "term_label": "nucleus",
  "gene_name": "Putative upstream-binding factor 1-like protein 6"
}